{
  "gene": "UniProtKB:Q7RTS1",
  "term_label": "nucleus",
  "term_id": "GO:0005634",
  "gene_name": "Class A basic helix-loop-helix protein 15",
  "gene_symbol": "BHLHA15"
}